alpha4-beta1 integrin-CD81 complex [GO:0070520] (cellular component) Definition: A protein complex that consists of an alpha4-beta1 integrin complex bound to membrane protein CD81, a member of the tetraspan family. Relationships: is_a GO:0098797 References: PMID:10229664, PMID:8757325 Also known as: ITGA4-ITGB1-CD81 complex